{
  "term_label": "aldehyde metabolic process",
  "gene_name": "Retinaldehyde dehydrogenase 3",
  "gene_symbol": "ALDH1A3",
  "term_id": "GO:0006081",
  "gene": "UniProtKB:P47895"
}